negative regulation of cardiac muscle tissue development [GO:0055026] (biological process) Definition: Any process that stops, prevents, or reduces the frequency, rate or extent of cardiac muscle tissue development. Sources: GOC:vk Relationships: is a type of GO:0045843; is a type of regulation of cardiac muscle tissue development [GO:0055024]; negatively regulates cardiac muscle tissue development [GO:0048738] Also known as: down regulation of cardiac muscle development, down-regulation of cardiac muscle development, downregulation of cardiac muscle development, negative regulation of heart muscle development, inhibition of cardiac muscle development